{
  "term_label": "Z disc",
  "gene": "UniProtKB:P50479",
  "gene_name": "PDZ and LIM domain protein 4",
  "gene_symbol": "PDLIM4",
  "term_id": "GO:0030018"
}